phosphatidylcholine-dolichol O-acyltransferase activity [GO:0047199] (molecular function) Definition: Catalysis of the reaction: 1,2-diacyl-sn-glycero-3-phosphocholine + dolichol = 1-acyl-sn-glycero-3-phosphocholine + acyldolichol. Sources: EC:2.3.1.83, RHEA:19285 Relationships: is a type of O-acyltransferase activity [GO:0008374] Also known as: 3-sn-phosphatidylcholine:dolichol O-acyltransferase activity